mannan metabolic process [GO:0010412] (biological process) Also known as: mannan metabolism Definition: The chemical reactions and pathways involving mannan, a group of polysaccharides containing a backbone composed of a polymer of D-mannose units. Relationships: is_a cell wall polysaccharide metabolic process [GO:0010383] Subtypes: mannan biosynthetic process [GO:0046354], mannan catabolic process [GO:0046355], beta-1,2-oligomannoside metabolic process [GO:0070135] Sources: GOC:tair_curators